{
  "gene_symbol": "LCP2",
  "gene": "UniProtKB:Q13094",
  "gene_name": "Lymphocyte cytosolic protein 2",
  "term_label": "protein-macromolecule adaptor activity",
  "term_id": "GO:0030674"
}